regulation of collagen biosynthetic process [GO:0032965] (biological process) Relationships: is_a regulation of biosynthetic process [GO:0009889]; is a type of GO:0010712; regulates GO:0032964 Sources: GOC:mah Also known as: regulation of collagen anabolism, regulation of collagen biosynthesis, regulation of collagen formation, regulation of collagen synthesis Subtypes: GO:0032966, positive regulation of collagen biosynthetic process [GO:0032967] Definition: Any process that modulates the frequency, rate or extent of the chemical reactions and pathways resulting in the formation of collagen, any of a group of fibrous proteins of very high tensile strength that form the main component of connective tissue in animals.